{
  "term_id": "GO:0031167",
  "gene_symbol": "NSUN4",
  "term_label": "rRNA methylation",
  "gene_name": "5-methylcytosine rRNA methyltransferase NSUN4",
  "gene": "UniProtKB:Q96CB9"
}